adenine nucleotide transmembrane transporter activity [GO:0000295] (molecular function) Definition: Enables the transfer of adenine nucleotides (AMP, ADP, and ATP) from one side of a membrane to the other. Subtypes: ATP transmembrane transporter activity [GO:0005347], ADP transmembrane transporter activity [GO:0015217], 3'-phosphoadenosine 5'-phosphosulfate transmembrane transporter activity [GO:0046964], NAD transmembrane transporter activity [GO:0051724], adenosine 3',5'-bisphosphate transmembrane transporter activity [GO:0071077], GO:0080122, cyclic-GMP-AMP transmembrane transporter activity [GO:0140360], GO:1902557 Relationships: is a type of purine nucleotide transmembrane transporter activity [GO:0015216]; is part of adenine nucleotide transport [GO:0051503] References: PMID:11566870